peptide hormone processing [GO:0016486] (biological process) Relationships: is a type of hormone metabolic process [GO:0042445]; is a type of amide metabolic process [GO:0043603]; is a type of GO:0140448 Sources: GOC:mah Definition: The generation of a mature peptide hormone by posttranslational processing of a prohormone. Regulation: regulated by regulation of peptide hormone processing [GO:0060568]; positively regulated by GO:0060569; negatively regulated by negative regulation of peptide hormone processing [GO:0060570] Subtypes: angiotensin maturation [GO:0002003], GO:0007225, insulin processing [GO:0030070], GO:0032455, GO:0034230, GO:0034231, endothelin maturation [GO:0034959], GO:0038004, glucagon processing [GO:0120116]